{
  "gene": "UniProtKB:P38646",
  "gene_symbol": "HSPA9",
  "gene_name": "Stress-70 protein, mitochondrial",
  "term_id": "GO:0031072",
  "term_label": "heat shock protein binding"
}